{
  "gene_name": "Transcription factor HES-1",
  "term_id": "GO:0009952",
  "term_label": "anterior/posterior pattern specification",
  "gene_symbol": "HES1",
  "gene": "UniProtKB:Q14469"
}